{
  "gene_name": "Bifunctional phosphoribosylaminoimidazole carboxylase_phosphoribosylaminoimidazole succinocarboxamide synthetase",
  "term_label": "cytosol",
  "gene": "UniProtKB:P22234",
  "gene_symbol": "PAICS",
  "term_id": "GO:0005829"
}